dolichyl-phosphate-mannose-protein mannosyltransferase activity [GO:0004169] (molecular function) Regulation: RO_0002211 by GO:0097713 Sources: EC:2.4.1.109, GOC:pr Also known as: O-glycoside mannosyltransferase, dolichyl-phosphate-mannose-protein O-mannosyltransferase activity, protein O-mannosyltransferase activity, dolichol phosphomannose-protein mannosyltransferase activity, dolichyl-phosphate-D-mannose:protein O-D-mannosyltransferase activity, protein O-D-mannosyltransferase activity Note: Note that this activity has never been observed in green plants. However, N- and C-mannosylation may occur in these species; see figure 1 in PMID:21558543. Relationships: is a type of mannosyltransferase activity [GO:0000030]; is a type of catalytic activity, acting on a protein [GO:0140096]; is part of protein O-linked glycosylation via mannose [GO:0035269] Definition: Catalysis of the reaction: dolichyl phosphate D-mannose + protein = dolichyl phosphate + O-D-mannosylprotein.